{
  "gene_name": "F-box_WD repeat-containing protein 8",
  "term_label": "protein ubiquitination",
  "gene": "UniProtKB:Q8N3Y1",
  "gene_symbol": "FBXW8",
  "term_id": "GO:0016567"
}